{
  "term_label": "membrane",
  "gene_symbol": "NIPAL2",
  "term_id": "GO:0016020",
  "gene_name": "NIPA-like protein 2",
  "gene": "UniProtKB:Q9H841"
}